alkyl hydroperoxide reductase complex [GO:0009321] (cellular component) Definition: An enzyme complex, usually a homodimer, which directly reduces cellular levels of organic hydroperoxides. Note: See also the molecular function term 'alkyl hydroperoxide reductase activity ; GO:0008785'. Relationships: is_a protein-containing complex [GO:0032991]; is part of cytoplasm [GO:0005737] References: PMID:2649484 Sources: GOC:jl